striated muscle cell apoptotic process [GO:0010658] (biological process) Sources: CL:0000737, GOC:dph, GOC:mtg_apoptosis, GOC:tb Regulation: RO_0002211 by regulation of striated muscle cell apoptotic process [GO:0010662]; positively regulated by positive regulation of striated muscle cell apoptotic process [GO:0010663]; negatively regulated by negative regulation of striated muscle cell apoptotic process [GO:0010664] Definition: A form of programmed cell death induced by external or internal signals that trigger the activity of proteolytic caspases, whose actions dismantle a striated muscle cell and result in its death. Striated muscle cells make up striated muscle fibers which are divided by transverse bands into striations. Also known as: striated muscle cell apoptosis Subtypes: GO:0010659 Relationships: is a type of muscle cell apoptotic process [GO:0010657]